{
  "term_label": "retinoic acid catabolic process",
  "gene_symbol": "CYP26A1",
  "term_id": "GO:0034653",
  "gene_name": "Cytochrome P450 26A1",
  "gene": "UniProtKB:O43174"
}